myotube differentiation [GO:0014902] (BP) Sources: GOC:mtg_muscle Definition: The process in which a relatively unspecialized cell acquires specialized features of a myotube cell. Myotube differentiation starts with myoblast fusion and the appearance of specific cell markers (this is the cell development step). Then individual myotubes can fuse to form bigger myotubes and start to contract. Myotubes are multinucleated cells that are formed when proliferating myoblasts exit the cell cycle, differentiate and fuse. Regulation: regulated by regulation of myotube differentiation [GO:0010830]; positively regulated by positive regulation of myotube differentiation [GO:0010831]; negatively regulated by negative regulation of myotube differentiation [GO:0010832] Subtypes: myotube differentiation involved in skeletal muscle regeneration [GO:0014908], skeletal muscle fiber differentiation [GO:0098528] Relationships: is a type of GO:0051146